positive regulation of cellular response to hypoxia [GO:1900039] (biological process) Also known as: activation of cellular response to hypoxic stress, activation of cellular response to lowered oxygen tension, positive regulation of cellular response to hypoxic stress, positive regulation of cellular response to lowered oxygen tension, up regulation of cellular response to hypoxic stress, up regulation of cellular response to lowered oxygen tension, up-regulation of cellular response to hypoxic stress, up-regulation of cellular response to lowered oxygen tension, upregulation of cellular response to hypoxic stress, upregulation of cellular response to lowered oxygen tension, activation of cellular response to hypoxia, up regulation of cellular response to hypoxia, up-regulation of cellular response to hypoxia, upregulation of cellular response to hypoxia Definition: Any process that activates or increases the frequency, rate or extent of cellular response to hypoxia. Sources: GOC:TermGenie, GOC:yaf Relationships: is a type of positive regulation of cellular process [GO:0048522]; is_a positive regulation of response to stimulus [GO:0048584]; is_a regulation of cellular response to hypoxia [GO:1900037]; positively regulates cellular response to hypoxia [GO:0071456]